clustering of voltage-gated sodium channels [GO:0045162] (biological process) Relationships: is a type of neuronal ion channel clustering [GO:0045161] Also known as: Nav channel clustering, clustering of voltage gated sodium channels, clustering of voltage-dependent sodium channels, voltage-gated sodium channel clustering References: PMID:11456440 Definition: The process in which voltage-gated sodium channels become localized together in high densities. In animals, nodes of Ranvier differ dramatically from internodal axonal regions in very high densities of voltage-dependent sodium (Nav) channels responsible for the rapid, inward ionic currents that produce membrane depolarization.